{
  "gene_symbol": "PTPRE",
  "gene": "UniProtKB:P23469",
  "term_id": "GO:0007165",
  "term_label": "signal transduction",
  "gene_name": "Receptor-type tyrosine-protein phosphatase epsilon"
}